negative regulation of locomotor rhythm [GO:1904060] (biological process) Definition: Any process that stops, prevents or reduces the frequency, rate or extent of locomotor rhythm. Also known as: down regulation of locomotor rhythm, down-regulation of locomotor rhythm, downregulation of locomotor rhythm, down regulation of circadian locomotor activity rhythm, down-regulation of circadian locomotor activity rhythm, downregulation of circadian locomotor activity rhythm, inhibition of circadian locomotor activity rhythm, inhibition of locomotor rhythm, negative regulation of circadian locomotor activity rhythm References: PMID:16310969 Sources: GOC:TermGenie, GO_REF:0000058 Relationships: is a type of negative regulation of circadian rhythm [GO:0042754]; is a type of negative regulation of behavior [GO:0048521]; is a type of regulation of locomotor rhythm [GO:1904059]; negatively regulates locomotor rhythm [GO:0045475]